{
  "gene": "UniProtKB:P13762",
  "gene_symbol": "HLA-DRB4",
  "term_id": "GO:0031902",
  "term_label": "late endosome membrane",
  "gene_name": "HLA class II histocompatibility antigen, DR beta 4 chain"
}